{
  "gene_name": "Thromboxane A2 receptor",
  "term_id": "GO:0045777",
  "gene": "UniProtKB:P21731",
  "gene_symbol": "TBXA2R",
  "term_label": "positive regulation of blood pressure"
}